mucus layer [GO:0070701] (cellular component) Definition: An extracellular region part that consists of a protective layer of mucus secreted by epithelial cells lining tubular organs of the body such as the colon or secreted into fluids such as saliva. Mucus is a viscous slimy secretion consisting of mucins (i.e. highly glycosylated mucin proteins) and various inorganic salts dissolved in water, with suspended epithelial cells and leukocytes. Also known as: extracellular proteinaceous gel, mucous, mucous layer, mucus Relationships: is a type of cellular anatomical structure [GO:0110165]; is part of extracellular region [GO:0005576] Subtypes: inner mucus layer [GO:0070702], GO:0070703 References: PMID:18806221, PMID:19432394 Sources: GOC:krc, GOC:mah, GOC:mm2, Wikipedia:Mucin